oxidative stress-induced premature senescence [GO:0090403] (biological process) Definition: A cellular senescence process associated with the dismantling of a cell as a response to oxidative stress, e.g. high levels of reactive oxygen species, such as superoxide anions, hydrogen peroxide, and hydroxyl radicals. Sources: GOC:BHF Relationships: is a type of stress-induced premature senescence [GO:0090400]; is part of GO:0034599